{
  "term_label": "ephrin receptor signaling pathway",
  "gene_name": "Ephrin type-A receptor 6",
  "gene": "UniProtKB:Q9UF33",
  "gene_symbol": "EPHA6",
  "term_id": "GO:0048013"
}